{
  "term_label": "Unknown biological process",
  "gene_name": "Taste receptor type 2 member 20",
  "term_id": "UNKNOWN:0002",
  "gene": "UniProtKB:P59543",
  "gene_symbol": "TAS2R20"
}